{
  "gene_symbol": "EDEM3",
  "term_label": "ubiquitin-dependent glycoprotein ERAD pathway",
  "gene_name": "ER degradation-enhancing alpha-mannosidase-like protein 3",
  "gene": "UniProtKB:Q9BZQ6",
  "term_id": "GO:0097466"
}